sinapoyltransferase activity [GO:0016752] (MF) Sources: GOC:ai Relationships: is a type of GO:0016747 Subtypes: O-sinapoyltransferase activity [GO:0016753] Definition: Catalysis of the transfer of a sinapoyl group to an acceptor molecule.